{
  "term_id": "UNKNOWN:0003",
  "gene_symbol": "A0A1W2PPM0",
  "gene": "UniProtKB:A0A1W2PPM0",
  "gene_name": "Uncharacterized protein",
  "term_label": "Unknown cellular component"
}